{
  "gene_name": "CUB and sushi domain-containing protein 1",
  "term_id": "UNKNOWN:0001",
  "gene": "UniProtKB:Q96PZ7",
  "term_label": "Unknown molecular function",
  "gene_symbol": "CSMD1"
}